Shc-EGFR complex [GO:0070435] (cellular component) Definition: A protein complex that contains the epidermal growth factor receptor (EGFR) and the adaptor protein Shc, and is involved in linking EGFR activation to the p21-Ras pathway. References: PMID:7798267 Sources: GOC:mah Also known as: Shc-Egfr complex, EGF stimulated Relationships: is_a plasma membrane protein complex [GO:0098797]